{
  "gene": "UniProtKB:Q8N8F7",
  "term_id": "UNKNOWN:0002",
  "gene_symbol": "LSMEM1",
  "term_label": "Unknown biological process",
  "gene_name": "Leucine-rich single-pass membrane protein 1"
}